{
  "gene_symbol": "MYO1C",
  "term_label": "plasma membrane",
  "gene": "UniProtKB:O00159",
  "gene_name": "Unconventional myosin-Ic",
  "term_id": "GO:0005886"
}